{
  "gene_symbol": "KRT5",
  "term_id": "GO:0030280",
  "term_label": "structural constituent of skin epidermis",
  "gene_name": "Keratin, type II cytoskeletal 5",
  "gene": "UniProtKB:P13647"
}